{
  "term_label": "protein serine/threonine kinase activity",
  "term_id": "GO:0004674",
  "gene_name": "Serine_threonine-protein kinase 3",
  "gene_symbol": "STK3",
  "gene": "UniProtKB:Q13188"
}